{
  "gene_name": "Double zinc ribbon and ankyrin repeat-containing protein 1",
  "term_label": "Unknown cellular component",
  "gene_symbol": "DZANK1",
  "term_id": "UNKNOWN:0003",
  "gene": "UniProtKB:Q9NVP4"
}